sn-glycerol 3-phosphate binding [GO:1902516] (molecular function) Definition: Binding to sn-glycerol 3-phosphate. Relationships: is a type of anion binding [GO:0043168]; is a type of GO:0097367 Note: An example of this is UgpB in E. coli [P0AG80] - see PMID:23013274. References: PMID:23013274 Sources: GOC:TermGenie, GOC:bhm